{
  "gene_name": "WD repeat and HMG-box DNA-binding protein 1",
  "gene": "UniProtKB:O75717",
  "gene_symbol": "WDHD1",
  "term_label": "chromatin binding",
  "term_id": "GO:0003682"
}